{
  "gene_symbol": "SLC38A5",
  "gene_name": "Sodium-coupled neutral amino acid transporter 5",
  "term_id": "GO:0032329",
  "term_label": "serine transport",
  "gene": "UniProtKB:Q8WUX1"
}